{
  "gene_name": "Interleukin-4",
  "gene": "UniProtKB:P05112",
  "gene_symbol": "IL4",
  "term_id": "GO:0050728",
  "term_label": "negative regulation of inflammatory response"
}